collateral sprouting of intact axon in response to injury [GO:0048673] (biological process) Definition: The process in which outgrowths develop from the axons of intact undamaged neurons as a result of injury to an axon. The collateral sprouts typically appear from undamaged axons in a tissue which has had part of its nerve supply removed, and they can often innervate successfully any cells that have lost some or all of their original synaptic input. Sources: GOC:dgh, GOC:dph, GOC:jid Relationships: is_a axon regeneration [GO:0031103]; is a type of collateral sprouting [GO:0048668] Regulation: regulated by regulation of collateral sprouting of intact axon in response to injury [GO:0048683]; positively regulated by positive regulation of collateral sprouting of intact axon in response to injury [GO:0048684]; negatively regulated by negative regulation of collateral sprouting of intact axon in response to injury [GO:0048685]